6-hydroxynicotinate 3-monooxygenase activity [GO:0043731] (molecular function) Relationships: is a type of oxidoreductase activity, acting on paired donors, with incorporation or reduction of molecular oxygen, NAD(P)H as one donor, and incorporation of one atom of oxygen [GO:0016709] Definition: Catalysis of the oxidative decarboxylation of 6-hydroxynicotinate to 2,5-dihydroxypyridine, dependent on O2, NADH +H+ and FAD. References: PMID:10091591 Sources: GOC:jl